seminal vesicle development [GO:0061107] (biological process) Sources: GOC:dph Relationships: is a type of reproductive structure development [GO:0048608]; is a type of GO:0048732 Definition: The progression of the seminal vesicle over time, from its formation to the mature structure. The seminal vesicle is a gland that contributes to the production of semen.